cell wall macromolecule metabolic process [GO:0044036] (biological process) Regulation: regulated by regulation of cell wall macromolecule metabolic process [GO:0010981] Definition: The chemical reactions and pathways involving macromolecules forming, or destined to form, part of the cell wall. A cell wall is a rigid or semi-rigid envelope lying outside the cell membrane of plant, fungal and most prokaryotic cells, maintaining their shape and protecting them from osmotic lysis. Sources: GOC:jl, GOC:mah Subtypes: cell wall polysaccharide metabolic process [GO:0010383], GO:0010384, cell wall macromolecule catabolic process [GO:0016998], GO:0044038 Relationships: is a type of macromolecule metabolic process [GO:0043170]; is part of cell wall organization or biogenesis [GO:0071554] Also known as: cellular cell wall macromolecule metabolic process, cellular cell wall macromolecule metabolism